{
  "gene_symbol": "B3GALT2",
  "gene_name": "Beta-1,3-galactosyltransferase 2",
  "term_label": "N-acetyl-beta-D-glucosaminide beta-(1,3)-galactosyltransferase activity",
  "gene": "UniProtKB:O43825",
  "term_id": "GO:0008499"
}